SC5b-7 complex [GO:0034995] (cellular component) Relationships: is a type of plasma membrane protein complex [GO:0098797] References: PMID:10090939 Definition: A protein complex that consist of complement components C5b6 and C7 stably inserted in a cell membrane. Formation of the SC5b-7 complex is the first phase of membrane attack complex assembly.